{
  "gene_symbol": "CRHR1",
  "term_label": "corticotropin-releasing hormone binding",
  "gene_name": "Corticotropin-releasing factor receptor 1",
  "gene": "UniProtKB:P34998",
  "term_id": "GO:0051424"
}